{
  "term_label": "immune response",
  "gene_symbol": "CCR8",
  "gene_name": "C-C chemokine receptor type 8",
  "term_id": "GO:0006955",
  "gene": "UniProtKB:P51685"
}